{
  "term_label": "calcium ion binding",
  "term_id": "GO:0005509",
  "gene_symbol": "KCNIP2",
  "gene": "UniProtKB:Q9NS61",
  "gene_name": "Kv channel-interacting protein 2"
}